{
  "gene_name": "Peripheral plasma membrane protein CASK",
  "term_id": "GO:0008104",
  "gene": "UniProtKB:O14936",
  "term_label": "intracellular protein localization",
  "gene_symbol": "CASK"
}